{
  "gene": "UniProtKB:Q8N5R6",
  "term_label": "Unknown biological process",
  "term_id": "UNKNOWN:0002",
  "gene_symbol": "CCDC33",
  "gene_name": "Coiled-coil domain-containing protein 33"
}